{
  "term_id": "GO:0051014",
  "term_label": "actin filament severing",
  "gene_name": "Protein flightless-1 homolog",
  "gene_symbol": "FLII",
  "gene": "UniProtKB:Q13045"
}